{
  "term_id": "GO:0001784",
  "gene_name": "Tyrosine-protein phosphatase non-receptor type 6",
  "term_label": "phosphotyrosine residue binding",
  "gene": "UniProtKB:P29350",
  "gene_symbol": "PTPN6"
}